short-chain fatty acid biosynthetic process [GO:0051790] (biological process) Subtypes: propionate biosynthetic process [GO:0019542], GO:0043441, butyrate biosynthetic process [GO:0046358], 2-oxobutyrate biosynthetic process [GO:0046360] Note: While there is not universal consensus on the lengths of short-, medium-, long- and very-long-chain fatty acids, the GO uses the definitions in ChEBI (see CHEBI:26666, CHEBI:59554, CHEBI:15904 and CHEBI:27283). Also known as: short chain fatty acid biosynthesis, short chain fatty acid biosynthetic process, short-chain fatty acid anabolism, short-chain fatty acid biosynthesis, short-chain fatty acid formation, short-chain fatty acid synthesis Relationships: is a type of GO:0006633; is a type of short-chain fatty acid metabolic process [GO:0046459] Definition: The chemical reactions and pathways resulting in the formation of a short-chain fatty acid. A short-chain fatty acid has an aliphatic tail containing fewer than 6 carbons. Sources: Wikipedia:Fatty_acid_metabolism